regulation of myeloid leukocyte differentiation [GO:0002761] (biological process) Subtypes: negative regulation of myeloid leukocyte differentiation [GO:0002762], positive regulation of myeloid leukocyte differentiation [GO:0002763], regulation of granulocyte differentiation [GO:0030852], regulation of macrophage differentiation [GO:0045649], regulation of monocyte differentiation [GO:0045655], regulation of osteoclast differentiation [GO:0045670], regulation of mast cell differentiation [GO:0060375] Relationships: is a type of regulation of myeloid cell differentiation [GO:0045637]; is a type of regulation of leukocyte differentiation [GO:1902105]; regulates GO:0002573 Definition: Any process that modulates the frequency, rate, or extent of myeloid leukocyte differentiation. Sources: GOC:add